{
  "term_label": "cytoplasm",
  "term_id": "GO:0005737",
  "gene": "UniProtKB:P61960",
  "gene_name": "Ubiquitin-fold modifier 1",
  "gene_symbol": "UFM1"
}